pyrogallol 1,2-oxygenase activity [GO:0050240] (molecular function) Definition: Catalysis of the reaction: O2 + pyrogallol = (Z)-5-oxohex-2-enedioate + 2 H+. Also known as: 1,2,3-trihydroxybenzene:oxygen 1,2-oxidoreductase (decyclizing), pyrogallol 1,2-dioxygenase activity Sources: EC:1.13.11.35, RHEA:19673 Relationships: is a type of GO:0016702